{
  "term_label": "glycerol-3-phosphate metabolic process",
  "gene": "UniProtKB:P21695",
  "gene_name": "Glycerol-3-phosphate dehydrogenase [NAD(+)], cytoplasmic",
  "term_id": "GO:0006072",
  "gene_symbol": "GPD1"
}